{
  "gene": "UniProtKB:Q8N143",
  "term_label": "nucleoplasm",
  "gene_symbol": "BCL6B",
  "gene_name": "B-cell CLL_lymphoma 6 member B protein",
  "term_id": "GO:0005654"
}